{
  "gene": "UniProtKB:Q00839",
  "term_label": "RNA binding",
  "gene_symbol": "HNRNPU",
  "term_id": "GO:0003723",
  "gene_name": "Heterogeneous nuclear ribonucleoprotein U"
}